menstrual cycle phase [GO:0022601] (biological process) Note: Note that this term should not be used for direct annotation. If you are trying to make an annotation to x phase, it is likely that the correct annotation is 'regulation of x/y phase transition' or to a process which occurs during the reported phase. To capture the phase when a specific location or process is observed, the phase term can be used in an annotation extension (PMID:24885854) applied to a cellular component term (with the relation exists_during) or a biological process term (with the relation happens_during). Subtypes: menarche [GO:0042696], menopause [GO:0042697], GO:0042703 Definition: The progression of physiological phases, occurring in the endometrium during the menstrual cycle that recur at regular intervals during the reproductive years. The menstrual cycle is an ovulation cycle where the endometrium is shed if pregnancy does not occur. Sources: GOC:dph, GOC:isa_complete, GOC:jid Relationships: is a type of biological phase [GO:0044848]